{
  "gene_symbol": "PTCD3",
  "term_id": "GO:0043024",
  "term_label": "ribosomal small subunit binding",
  "gene": "UniProtKB:Q96EY7",
  "gene_name": "Small ribosomal subunit protein mS39"
}